{
  "gene_symbol": "DNAJA4",
  "term_label": "protein refolding",
  "gene": "UniProtKB:Q8WW22",
  "gene_name": "DnaJ homolog subfamily A member 4",
  "term_id": "GO:0042026"
}